{
  "gene_symbol": "GUCD1",
  "term_label": "Unknown biological process",
  "gene": "UniProtKB:Q96NT3",
  "gene_name": "Protein GUCD1",
  "term_id": "UNKNOWN:0002"
}